{
  "gene_name": "Ribosomal protein uL30-like",
  "gene_symbol": "RPL7L1",
  "gene": "UniProtKB:Q6DKI1",
  "term_id": "GO:0022625",
  "term_label": "cytosolic large ribosomal subunit"
}